{
  "gene_symbol": "FBXO6",
  "term_id": "GO:0031146",
  "term_label": "SCF-dependent proteasomal ubiquitin-dependent protein catabolic process",
  "gene_name": "F-box only protein 6",
  "gene": "UniProtKB:Q9NRD1"
}